{
  "gene": "UniProtKB:A0A0A0MRZ7",
  "term_id": "GO:0006955",
  "gene_name": "Immunoglobulin kappa variable 2D-26",
  "term_label": "immune response",
  "gene_symbol": "IGKV2D-26"
}